{
  "gene_name": "Deubiquitinase DESI2",
  "gene": "UniProtKB:Q9BSY9",
  "term_id": "GO:0101005",
  "gene_symbol": "DESI2",
  "term_label": "deubiquitinase activity"
}